{
  "term_label": "Unknown molecular function",
  "gene": "UniProtKB:Q6ZW76",
  "term_id": "UNKNOWN:0001",
  "gene_symbol": "ANKS3",
  "gene_name": "Ankyrin repeat and SAM domain-containing protein 3"
}